{
  "gene_symbol": "NPIPA3",
  "gene": "UniProtKB:F8WFD2",
  "gene_name": "Nuclear pore complex-interacting protein family member A3",
  "term_label": "Unknown biological process",
  "term_id": "UNKNOWN:0002"
}